{
  "gene": "UniProtKB:Q13615",
  "gene_symbol": "MTMR3",
  "term_id": "GO:0005737",
  "term_label": "cytoplasm",
  "gene_name": "Myotubularin-related protein 3"
}